{
  "gene_name": "Taste receptor type 2 member 40",
  "gene_symbol": "TAS2R40",
  "term_id": "GO:0033038",
  "gene": "UniProtKB:P59535",
  "term_label": "bitter taste receptor activity"
}